UDP-N-acetylgalactosamine biosynthetic process [GO:0019277] (BP) Also known as: UDP-N-acetylgalactosamine anabolism, UDP-N-acetylgalactosamine biosynthesis, UDP-N-acetylgalactosamine formation, UDP-N-acetylgalactosamine synthesis Definition: The chemical reactions and pathways resulting in the formation of UDP-N-acetylgalactosamine, a substance composed of N-acetylgalactosamine, a common structural unit of oligosaccharides, in glycosidic linkage with uridine diphosphate. Relationships: is_a nucleotide-sugar biosynthetic process [GO:0009226]; is_a UDP-N-acetylgalactosamine metabolic process [GO:0019276]; is a type of amino sugar biosynthetic process [GO:0046349] Sources: GOC:ai